{
  "gene_symbol": "TAF9",
  "gene_name": "Transcription initiation factor TFIID subunit 9",
  "term_id": "GO:0051123",
  "term_label": "RNA polymerase II preinitiation complex assembly",
  "gene": "UniProtKB:Q16594"
}